{
  "gene_name": "Ephrin type-A receptor 1",
  "gene": "UniProtKB:P21709",
  "gene_symbol": "EPHA1",
  "term_label": "plasma membrane",
  "term_id": "GO:0005886"
}